{
  "gene": "UniProtKB:Q8IYI8",
  "gene_symbol": "ZNF440",
  "gene_name": "Zinc finger protein 440",
  "term_id": "GO:0005634",
  "term_label": "nucleus"
}